{
  "term_id": "GO:0014820",
  "gene_symbol": "MYLK",
  "gene": "UniProtKB:Q15746",
  "term_label": "tonic smooth muscle contraction",
  "gene_name": "Myosin light chain kinase, smooth muscle"
}